retinal rod cell apoptotic process [GO:0097473] (biological process) References: PMID:17202487 Sources: CL:0000604, GOC:jc Relationships: is a type of neuron apoptotic process [GO:0051402]; is a type of GO:1990009 Also known as: rod photoreceptor apoptotic process Definition: Any apoptotic process in a retinal rod cell, one of the two photoreceptor cell types of the vertebrate retina.